{
  "gene_symbol": "ARHGAP6",
  "term_label": "actin filament organization",
  "gene_name": "Rho GTPase-activating protein 6",
  "term_id": "GO:0007015",
  "gene": "UniProtKB:O43182"
}